negative regulation of asperfuranone biosynthetic process [GO:1900638] (biological process) Sources: GOC:TermGenie, GOC:di Relationships: is a type of regulation of asperfuranone biosynthetic process [GO:1900637]; is a type of negative regulation of polyketide biosynthetic process [GO:1900733]; is a type of negative regulation of alcohol biosynthetic process [GO:1902931]; negatively regulates asperfuranone biosynthetic process [GO:1900554] Definition: Any process that stops, prevents or reduces the frequency, rate or extent of asperfuranone biosynthetic process. Also known as: down regulation of asperfuranone anabolism, down regulation of asperfuranone biosynthesis, down regulation of asperfuranone biosynthetic process, down regulation of asperfuranone formation, down regulation of asperfuranone synthesis, down-regulation of asperfuranone anabolism, down-regulation of asperfuranone biosynthesis, down-regulation of asperfuranone biosynthetic process, down-regulation of asperfuranone formation, down-regulation of asperfuranone synthesis, downregulation of asperfuranone anabolism, downregulation of asperfuranone biosynthesis, downregulation of asperfuranone biosynthetic process, downregulation of asperfuranone formation, downregulation of asperfuranone synthesis, inhibition of asperfuranone anabolism, inhibition of asperfuranone biosynthesis, inhibition of asperfuranone formation, inhibition of asperfuranone synthesis, negative regulation of asperfuranone anabolism, negative regulation of asperfuranone biosynthesis, negative regulation of asperfuranone formation, negative regulation of asperfuranone synthesis, inhibition of asperfuranone biosynthetic process